{
  "gene": "UniProtKB:P01717",
  "term_id": "GO:0019814",
  "gene_name": "Immunoglobulin lambda variable 3-25",
  "term_label": "immunoglobulin complex",
  "gene_symbol": "IGLV3-25"
}